{
  "term_label": "Unknown molecular function",
  "gene": "UniProtKB:P43243",
  "gene_symbol": "MATR3",
  "term_id": "UNKNOWN:0001",
  "gene_name": "Matrin-3"
}